{
  "gene_name": "Transcription factor E2-alpha",
  "gene": "UniProtKB:P15923",
  "term_id": "GO:0006357",
  "gene_symbol": "TCF3",
  "term_label": "regulation of transcription by RNA polymerase II"
}